negative regulation of smooth muscle contraction [GO:0045986] (biological process) Relationships: is a type of regulation of smooth muscle contraction [GO:0006940]; is_a negative regulation of muscle contraction [GO:0045932]; negatively regulates smooth muscle contraction [GO:0006939] Also known as: down regulation of smooth muscle contraction, down-regulation of smooth muscle contraction, downregulation of smooth muscle contraction, inhibition of smooth muscle contraction, smooth muscle relaxation Subtypes: smooth muscle relaxation of the bladder outlet [GO:0060085], GO:0060087, GO:0060451, negative regulation of uterine smooth muscle contraction [GO:0070473], negative regulation of gastro-intestinal system smooth muscle contraction [GO:1904305], negative regulation of smooth muscle contraction involved in micturition [GO:1904319], negative regulation of vascular associated smooth muscle contraction [GO:1904694] Definition: Any process that stops, prevents, or reduces the frequency, rate or extent of smooth muscle contraction. Sources: GOC:go_curators